{
  "gene": "UniProtKB:O75159",
  "term_label": "Unknown molecular function",
  "gene_name": "Suppressor of cytokine signaling 5",
  "gene_symbol": "SOCS5",
  "term_id": "UNKNOWN:0001"
}